right caudal flagellum [GO:0097561] (cellular component) References: PMID:16607022, PMID:5961344 Sources: GOC:giardia, ISBN:9780124260207 Definition: A cilium (also called flagellum) found in Giardia species (trophozoite stage). It is nucleated by the right caudal basal body, extending cytoplasmically and exiting at the posterior end of the cell body. Also known as: right caudal cilium Relationships: is a type of 9+2 motile cilium [GO:0097729] Note: Note that we deem cilium and microtubule-based flagellum to be equivalent; the primary term name reflects frequency of use. Also note that, due to the asymmetric nature of the Giardia trophozoite, this term is defined spatially as the trophozoite is viewed from the dorsal side, with the two nuclei dorsal to the ventral disc, and the ventral disc toward the anterior.